{
  "term_label": "plasma membrane",
  "gene": "UniProtKB:O75106",
  "term_id": "GO:0005886",
  "gene_name": "Retina-specific copper amine oxidase",
  "gene_symbol": "AOC2"
}